{
  "term_id": "GO:2000812",
  "gene_symbol": "ASB2",
  "gene": "UniProtKB:Q96Q27",
  "term_label": "regulation of barbed-end actin filament capping",
  "gene_name": "Ankyrin repeat and SOCS box protein 2"
}